cleavage body [GO:0071920] (cellular component) Relationships: is a type of nuclear body [GO:0016604] References: PMID:10564273, PMID:11598190, PMID:8654386 Definition: A nuclear body that contains proteins involved in pre-mRNA 3'-end cleavage and polyadenylation, such as DDX1, CSTF2 and CPSFs, as well as the transcription factors TFIIE and TFIIF. Cleavage bodies are localized adjacent to Cajal bodies and are involved in mRNA3'-end processing.